{
  "gene": "UniProtKB:Q66K74",
  "gene_symbol": "MAP1S",
  "gene_name": "Microtubule-associated protein 1S",
  "term_id": "GO:0005829",
  "term_label": "cytosol"
}